{
  "gene": "UniProtKB:Q9BXJ1",
  "gene_symbol": "C1QTNF1",
  "term_label": "Unknown molecular function",
  "gene_name": "Complement C1q tumor necrosis factor-related protein 1",
  "term_id": "UNKNOWN:0001"
}